{
  "gene_symbol": "RYR1",
  "gene": "UniProtKB:P21817",
  "term_label": "calcium channel complex",
  "gene_name": "Ryanodine receptor 1",
  "term_id": "GO:0034704"
}